{
  "gene": "UniProtKB:P35858",
  "gene_symbol": "IGFALS",
  "term_label": "Unknown biological process",
  "gene_name": "Insulin-like growth factor-binding protein complex acid labile subunit",
  "term_id": "UNKNOWN:0002"
}